{
  "gene_name": "Prostate stem cell antigen",
  "term_id": "GO:0005886",
  "term_label": "plasma membrane",
  "gene_symbol": "PSCA",
  "gene": "UniProtKB:O43653"
}